bract formation [GO:0010434] (biological process) Relationships: is a type of plant organ formation [GO:1905393]; is part of bract morphogenesis [GO:0010433] Definition: The process that gives rise to a bract. This process pertains to the initial formation of a structure from unspecified parts. A bract is a leaf, usually different in form from the foliage leaves, subtending a flower or inflorescence. References: PMID:16554366 Sources: GOC:tb, PO:0009055